{
  "gene_name": "Galactosylceramide sulfotransferase",
  "gene_symbol": "GAL3ST1",
  "term_id": "GO:0001733",
  "term_label": "galactosylceramide sulfotransferase activity",
  "gene": "UniProtKB:Q99999"
}